mesonephric juxtaglomerular apparatus development [GO:0061212] (biological process) Relationships: is a type of juxtaglomerular apparatus development [GO:0072051]; is part of mesonephros development [GO:0001823] Definition: The process whose specific outcome is the progression of the juxtaglomerular apparatus in the mesonephros over time, from its formation to the mature structure. The juxtaglomerular apparatus is an anatomical structure which consists of juxtaglomerular cells, extraglomerular mesangial cells and the macula densa. The juxtaglomerular apparatus lies adjacent to the glomerulus and regulates kidney function by maintaining the blood flow to the kidney and the filtration rate. Sources: GOC:mtg_kidney_jan10